{
  "gene": "UniProtKB:Q58FF7",
  "term_id": "GO:0051082",
  "gene_symbol": "HSP90AB3P",
  "term_label": "unfolded protein binding",
  "gene_name": "Putative heat shock protein HSP 90-beta-3"
}